{
  "gene_symbol": "PPIL1",
  "term_label": "peptidyl-prolyl cis-trans isomerase activity",
  "gene": "UniProtKB:Q9Y3C6",
  "gene_name": "Peptidyl-prolyl cis-trans isomerase-like 1",
  "term_id": "GO:0003755"
}